response to oxygen-containing compound [GO:1901700] (biological process) Relationships: is a type of response to chemical [GO:0042221] Definition: Any process that results in a change in state or activity of a cell or an organism (in terms of movement, secretion, enzyme production, gene expression, etc.) as a result of an oxygen-containing compound stimulus. Also known as: response to oxygen molecular entity Note: Note that this term is in the subset of terms that should not be used for direct gene product annotation. Instead, select a child term or, if no appropriate child term exists, please request a new term. Direct annotations to this term may be amended during annotation QC. Sources: GOC:TermGenie, GOC:pr Subtypes: GO:0000302, GO:0009415, response to gibberellin [GO:0009739], GO:0009741, GO:0009743, GO:0009751, GO:0009961, GO:0010034, response to carbon dioxide [GO:0010037], response to chlorate [GO:0010157], response to nitrate [GO:0010167], response to chitin [GO:0010200], GO:0010238, response to sulfur dioxide [GO:0010477], response to brefeldin A [GO:0031001], response to methotrexate [GO:0031427], response to estradiol [GO:0032355], response to peptidoglycan [GO:0032494], response to muramyl dipeptide [GO:0032495], response to lipopolysaccharide [GO:0032496], response to retinoic acid [GO:0032526], response to hydroperoxide [GO:0033194], response to vitamin E [GO:0033197], response to ATP [GO:0033198], response to vitamin B2 [GO:0033274], response to vitamin D [GO:0033280], response to cobalamin [GO:0033590], response to triglyceride [GO:0034014], response to silicon dioxide [GO:0034021], response to carbon monoxide [GO:0034465], response to vitamin B6 [GO:0034516], GO:0034697, response to nitrogen dioxide [GO:0035713], response to trichostatin A [GO:0035983], GO:0036272, response to statin [GO:0036273], response to lapatinib [GO:0036274], response to ximelagatran [GO:0036288], response to sterol [GO:0036314], GO:0042220, GO:0043201, response to peptide hormone [GO:0043434], response to amylopectin [GO:0044591], GO:0045472, response to bacteriocin [GO:0046678], response to carbamate [GO:0046681], response to chromate [GO:0046687], response to tellurium ion [GO:0046690], response to cAMP [GO:0051591], GO:0051593, response to cGMP [GO:0070305], GO:0070391, response to fatty acid [GO:0070542], response to biotin [GO:0070781], response to heparin [GO:0071503], response to mycophenolic acid [GO:0071505], response to nitric oxide [GO:0071731], response to catecholamine [GO:0071869], response to methyl methanesulfonate [GO:0072702], response to sodium dodecyl sulfate [GO:0072706], response to selenite ion [GO:0072714], response to actinomycin D [GO:0072716], response to dithiothreitol [GO:0072720], response to 4-nitroquinoline N-oxide [GO:0072724], response to papulacandin B [GO:0072730], GO:0080021, response to indolebutyric acid [GO:0080026], GO:0080033, GO:0080052, response to phenylalanine [GO:0080053], GO:0080094, response to thyroxine [GO:0097068], response to alcohol [GO:0097305], response to N-acetyl-D-glucosamine [GO:0097315], response to 5-fluoro-2'-deoxyuridine [GO:0097330], response to risperidone [GO:0097336], GO:1901322, GO:1901323, GO:1901325, GO:1901327, GO:1901328, response to L-thialysine [GO:1901345], response to L-canavanine [GO:1901354], response to L-cysteine [GO:1901367], response to glutathione [GO:1901370], response to formic acid [GO:1901425], GO:1901426, response to paracetamol [GO:1901554], response to candesartan [GO:1901556], response to ribavirin [GO:1901559], GO:1901593, response to capsazepine [GO:1901594], GO:1901595, GO:1901596, response to carbendazim [GO:1901597], GO:1901654, cellular response to oxygen-containing compound [GO:1901701], response to L-glutamate [GO:1902065], GO:1902111, GO:1902140, response to strigolactone [GO:1902347], response to vanadate(3-) [GO:1902438], GO:1903412, response to glycoside [GO:1903416], response to acetylsalicylate [GO:1903492], response to clopidogrel [GO:1903493], GO:1903576, response to arsenite(3-) [GO:1903840], response to arsenite ion [GO:1903842], response to bisphenol A [GO:1903925], response to acrylamide [GO:1903937], response to micafungin [GO:1903967], GO:1904014, response to acadesine [GO:1904101], response to cordycepin [GO:1904309], response to kainic acid [GO:1904373], response to formaldehyde [GO:1904404], response to D-galactosamine [GO:1904421], response to L-dopa [GO:1904473], response to tetrahydrofolate [GO:1904481], GO:1904565, response to glycoprotein [GO:1904587], response to resveratrol [GO:1904638], response to methionine [GO:1904640], response to dinitrophenol [GO:1904641], response to amyloid-beta [GO:1904645], response to nitroglycerin [GO:1904842], GO:1904844, response to bleomycin [GO:1904975], response to acetylcholine [GO:1905144], response to cyclosporin A [GO:1905237], GO:1905242, response to homocysteine [GO:1905374], response to flavonoid [GO:1905395], response to glycine [GO:1905429], response to chondroitin 6'-sulfate [GO:1905439], GO:1905441, response to acetaldehyde [GO:1905640], response to phosphatidylethanolamine [GO:1905711], response to puromycin [GO:1905794], response to pyrimidine ribonucleotide [GO:1905834], response to temozolomide [GO:1990054]